{
  "gene_name": "CMRF35-like molecule 6",
  "term_id": "GO:0045088",
  "term_label": "regulation of innate immune response",
  "gene_symbol": "CD300C",
  "gene": "UniProtKB:Q08708"
}